{
  "gene_name": "Snurportin-1",
  "term_label": "Unknown cellular component",
  "term_id": "UNKNOWN:0003",
  "gene": "UniProtKB:O95149",
  "gene_symbol": "SNUPN"
}